{
  "gene_symbol": "PIK3R1",
  "term_label": "phosphatidylinositol 3-kinase complex, class IA",
  "gene": "UniProtKB:P27986",
  "term_id": "GO:0005943",
  "gene_name": "Phosphatidylinositol 3-kinase regulatory subunit alpha"
}